{
  "term_label": "catalytic step 2 spliceosome",
  "gene_name": "Protein FRG1",
  "term_id": "GO:0071013",
  "gene_symbol": "FRG1",
  "gene": "UniProtKB:Q14331"
}